{
  "term_id": "GO:0015459",
  "gene_symbol": "SGK2",
  "gene_name": "Serine_threonine-protein kinase Sgk2",
  "gene": "UniProtKB:Q9HBY8",
  "term_label": "potassium channel regulator activity"
}